aphidicolan-16 beta-ol synthase activity [GO:0046567] (molecular function) Definition: Catalysis of the reaction: 9-alpha-copalyl diphosphate + H2O = aphidicolan-16-beta-ol + diphosphate. Also known as: 9-alpha-copalyl-diphosphate diphosphate-lyase (aphidicolan-16-beta-ol-forming) References: PMID:12149019 Sources: EC:4.2.3.42 Relationships: is_a carbon-oxygen lyase activity, acting on phosphates [GO:0016838]